borate export across plasma membrane [GO:0140159] (biological process) Definition: The directed movement of borate from inside of a cell, across the plasma membrane and into the extracellular region. References: PMID:17459946 Sources: GOC:vw Relationships: is_a borate transmembrane transport [GO:0035445]; is a type of GO:0140115